{
  "gene_symbol": "TNNC1",
  "gene_name": "Troponin C, slow skeletal and cardiac muscles",
  "gene": "UniProtKB:P63316",
  "term_id": "GO:0005509",
  "term_label": "calcium ion binding"
}